{
  "term_label": "axon development",
  "gene": "UniProtKB:O75312",
  "gene_name": "Zinc finger protein ZPR1",
  "term_id": "GO:0061564",
  "gene_symbol": "ZPR1"
}